{
  "gene_name": "Cyclin-dependent kinases regulatory subunit 1",
  "gene_symbol": "CKS1B",
  "term_label": "histone binding",
  "term_id": "GO:0042393",
  "gene": "UniProtKB:P61024"
}